{
  "gene_symbol": "CNPY4",
  "term_label": "signaling receptor binding",
  "gene_name": "Protein canopy homolog 4",
  "term_id": "GO:0005102",
  "gene": "UniProtKB:Q8N129"
}